regulation of mesenchymal cell apoptotic process involved in metanephric nephron morphogenesis [GO:0072304] (biological process) Definition: Any process that modulates the occurrence or rate of mesenchymal stem cell death by apoptotic process that contributes to the shaping of the nephron in the metanephros. Also known as: regulation of mesenchymal stem cell apoptotic process involved in metanephric nephron morphogenesis, regulation of mesenchymal stem cell apoptosis involved in metanephric nephron morphogenesis Relationships: is a type of regulation of mesenchymal cell apoptotic process involved in nephron morphogenesis [GO:0072039]; is a type of regulation of mesenchymal cell apoptotic process involved in metanephros development [GO:1900211]; regulates mesenchymal stem cell maintenance involved in metanephric nephron morphogenesis [GO:0072309]; RO_0002211 mesenchymal cell apoptotic process involved in metanephric nephron morphogenesis [GO:1901147] Subtypes: negative regulation of mesenchymal cell apoptotic process involved in metanephric nephron morphogenesis [GO:0072305], positive regulation of mesenchymal cell apoptotic process involved in metanephric nephron morphogenesis [GO:0072306] Sources: GOC:mtg_apoptosis, GOC:mtg_kidney_jan10